{
  "term_id": "GO:0030100",
  "term_label": "regulation of endocytosis",
  "gene": "UniProtKB:P61018",
  "gene_name": "Ras-related protein Rab-4B",
  "gene_symbol": "RAB4B"
}